{
  "gene_name": "Hydroxyacylglutathione hydrolase, mitochondrial",
  "term_label": "hydroxyacylglutathione hydrolase activity",
  "term_id": "GO:0004416",
  "gene_symbol": "HAGH",
  "gene": "UniProtKB:Q16775"
}